{
  "gene_name": "Pancreatic secretory granule membrane major glycoprotein GP2",
  "gene": "UniProtKB:P55259",
  "term_id": "GO:0005615",
  "gene_symbol": "GP2",
  "term_label": "extracellular space"
}